{
  "gene_name": "Phosphatidylinositol 4-kinase beta",
  "term_id": "GO:0048839",
  "term_label": "inner ear development",
  "gene_symbol": "PI4KB",
  "gene": "UniProtKB:Q9UBF8"
}